rhamnogalacturonan I metabolic process [GO:0010395] (biological process) Definition: The chemical reactions and pathways involving rhamnogalacturonan I (RGI), a branched pectin with a backbone of alternating alpha-(1->2)-linked rhamnose and alpha-(1->4)-linked D-galacturonic acid residues that carries neutral side-chains of predominantly beta-(1->4)-D-galactose and/or alpha-(1->5)-L-arabinose residues attached to the rhamnose residues of the RGI backbone. Sources: GOC:tair_curators Also known as: rhamnogalacturonan I metabolism, RGI metabolism Relationships: is a type of cell wall polysaccharide metabolic process [GO:0010383]; is_a cell wall pectin metabolic process [GO:0052546] Subtypes: rhamnogalacturonan I biosynthetic process [GO:0010246], rhamnogalacturonan I side chain metabolic process [GO:0010400]